{
  "term_id": "UNKNOWN:0003",
  "gene_name": "Putative uncharacterized protein encoded by LINC00114",
  "gene_symbol": "LINC00114",
  "gene": "UniProtKB:Q6XXX2",
  "term_label": "Unknown cellular component"
}